{
  "term_label": "axon guidance",
  "gene_name": "Cyclin-dependent kinase 5 activator 2",
  "term_id": "GO:0007411",
  "gene": "UniProtKB:Q13319",
  "gene_symbol": "CDK5R2"
}